{
  "gene_symbol": "KLHDC4",
  "term_id": "UNKNOWN:0002",
  "gene_name": "Kelch domain-containing protein 4",
  "term_label": "Unknown biological process",
  "gene": "UniProtKB:Q8TBB5"
}